{
  "term_label": "chloride channel activity",
  "term_id": "GO:0005254",
  "gene_symbol": "GABRP",
  "gene_name": "Gamma-aminobutyric acid receptor subunit pi",
  "gene": "UniProtKB:O00591"
}